prostanoid receptor activity [GO:0004954] (molecular function) Definition: Combining with a prostanoid, any compound based on or derived from the prostanoate structure, to initiate a change in cell activity. Relationships: is a type of icosanoid receptor activity [GO:0004953] Sources: ISBN:0198506732 Subtypes: prostaglandin receptor activity [GO:0004955], thromboxane receptor activity [GO:0004960]